carbon catabolite repression [GO:0061985] (BP) Relationships: is a type of catabolite repression [GO:0061984] Subtypes: carbon catabolite repression of transcription [GO:0045013] Definition: A process in which the presence of one carbon source leads to the modulation of the frequency, rate, or extent of the metabolism of other carbon sources. References: PMID:29295552